{
  "gene_symbol": "BCAT2",
  "gene": "UniProtKB:O15382",
  "term_label": "mitochondrion",
  "gene_name": "Branched-chain-amino-acid aminotransferase, mitochondrial",
  "term_id": "GO:0005739"
}